peptidoglycan peptide transmembrane transporter activity [GO:0015640] (molecular function) Relationships: is a type of peptidoglycan transmembrane transporter activity [GO:0015647]; is part of GO:0015834 Definition: Enables the transfer of peptidoglycan peptides from one side of a membrane to the other. Peptidoglycan peptides are the oligopeptides found in peptidoglycan networks which cross-link the polysaccharide chains. Sources: ISBN:0198506732 Also known as: murein peptide transporter activity, muropeptide transporter activity